{
  "term_id": "UNKNOWN:0003",
  "gene_name": "Tumor necrosis factor receptor superfamily member 13B",
  "gene": "UniProtKB:O14836",
  "term_label": "Unknown cellular component",
  "gene_symbol": "TNFRSF13B"
}